Vps55/Vps68 complex [GO:0034424] (cellular component) References: PMID:18216282 Definition: A membrane-associated protein complex that is required for a late stage of endosomal transport. In budding yeast, this complex consists of Vps55p and Vps68p proteins. Relationships: is_a membrane protein complex [GO:0098796]; is part of endosome membrane [GO:0010008]